{
  "gene_symbol": "RPS7",
  "term_label": "rRNA processing",
  "gene_name": "Small ribosomal subunit protein eS7",
  "gene": "UniProtKB:P62081",
  "term_id": "GO:0006364"
}